{
  "gene": "UniProtKB:Q9UJ90",
  "gene_symbol": "KCNE5",
  "term_label": "ventricular cardiac muscle cell action potential",
  "gene_name": "Potassium voltage-gated channel subfamily E regulatory beta subunit 5",
  "term_id": "GO:0086005"
}